{
  "term_id": "GO:0016020",
  "term_label": "membrane",
  "gene_symbol": "SLC15A4",
  "gene": "UniProtKB:Q8N697",
  "gene_name": "Solute carrier family 15 member 4"
}